{
  "gene": "UniProtKB:O95847",
  "term_label": "mitochondrial inner membrane",
  "gene_name": "Mitochondrial uncoupling protein 4",
  "gene_symbol": "SLC25A27",
  "term_id": "GO:0005743"
}